{
  "gene_name": "Galectin-related protein",
  "term_id": "GO:0030246",
  "term_label": "carbohydrate binding",
  "gene": "UniProtKB:Q3ZCW2",
  "gene_symbol": "LGALSL"
}